{
  "term_id": "GO:0070740",
  "gene_symbol": "TTLL13",
  "gene": "UniProtKB:A6NNM8",
  "gene_name": "Tubulin polyglutamylase TTLL13",
  "term_label": "tubulin-glutamic acid ligase activity"
}